ubiquitin binding [GO:0043130] (MF) Subtypes: linear polyubiquitin binding [GO:1990450] Definition: Binding to ubiquitin, a protein that when covalently bound to other cellular proteins marks them for proteolytic degradation. Relationships: is a type of GO:0032182 Sources: GOC:ecd